{
  "term_label": "Unknown cellular component",
  "term_id": "UNKNOWN:0003",
  "gene_name": "T cell receptor alpha variable 21",
  "gene_symbol": "TRAV21",
  "gene": "UniProtKB:A0A0B4J279"
}